Isw1 complex [GO:0016587] (cellular component) References: PMID:15020051, PMID:15284901, PMID:16568949, PMID:21810179 Sources: GOC:krc, GOC:mah Subtypes: Isw1a complex [GO:0036436], GO:0036437 Definition: A protein complex that contains an Isw1 subunit from the ISWI-family of ATPases and acts to modify chromatin structure. Relationships: is a type of ISWI-type complex [GO:0031010]